DnaA-Hda complex [GO:1990083] (cellular component) Relationships: is a type of replication inhibiting complex [GO:1990078] Definition: A protein complex that inactivates the function of DnaA by inhibiting the phosphorylation of DnaA-ADP to DnaA-ATP and thereby preventing multiple events of replication initiation. In E. coli, this complex is composed of DnaA and Hda. References: PMID:21708944 Sources: GOC:bhm